{
  "term_id": "GO:0005886",
  "gene_name": "Dystrobrevin beta",
  "gene_symbol": "DTNB",
  "gene": "UniProtKB:O60941",
  "term_label": "plasma membrane"
}